regulation of cortisol secretion [GO:0051462] (biological process) Definition: Any process that modulates the frequency, rate or extent of the regulated release of cortisol from a cell. Sources: GOC:ai Relationships: is a type of regulation of glucocorticoid secretion [GO:2000849]; regulates GO:0043400 Subtypes: negative regulation of cortisol secretion [GO:0051463], positive regulation of cortisol secretion [GO:0051464]